{
  "term_id": "GO:0009897",
  "gene_name": "Putative high affinity immunoglobulin gamma Fc receptor IB",
  "gene_symbol": "FCGR1BP",
  "gene": "UniProtKB:Q92637",
  "term_label": "external side of plasma membrane"
}